positive regulation of glyoxylate cycle [GO:2000876] (BP) Sources: GOC:dgf Relationships: is a type of positive regulation of carbohydrate metabolic process [GO:0045913]; is_a GO:0062013; is a type of regulation of glyoxylate cycle [GO:2000874]; positively regulates glyoxylate cycle [GO:0006097] Definition: Any process that activates or increases the frequency, rate or extent of glyoxylate cycle. Also known as: positive regulation of glyoxylate bypass